{
  "gene_symbol": "LNX2",
  "term_label": "Unknown biological process",
  "gene": "UniProtKB:Q8N448",
  "term_id": "UNKNOWN:0002",
  "gene_name": "Ligand of Numb protein X 2"
}